{
  "term_id": "GO:0008021",
  "gene_symbol": "CLCN5",
  "term_label": "synaptic vesicle",
  "gene": "UniProtKB:P51795",
  "gene_name": "H(+)_Cl(-) exchange transporter 5"
}